{
  "gene": "UniProtKB:Q9Y4A5",
  "gene_name": "Transformation_transcription domain-associated protein",
  "term_id": "GO:0035267",
  "gene_symbol": "TRRAP",
  "term_label": "NuA4 histone acetyltransferase complex"
}